{
  "term_label": "1-phosphatidylinositol-5-kinase activity",
  "gene": "UniProtKB:Q9Y2I7",
  "gene_symbol": "PIKFYVE",
  "term_id": "GO:0052810",
  "gene_name": "1-phosphatidylinositol 3-phosphate 5-kinase"
}